pyrroline-2-carboxylate reductase activity [GO:0050241] (molecular function) Also known as: L-proline:NAD(P)+ 2-oxidoreductase activity, delta1-pyrroline-2-carboxylate reductase activity Definition: Catalysis of the reaction: L-proline + NAD(P)+ = 1-pyrroline-2-carboxylate + NAD(P)H + H+. Relationships: is a type of oxidoreductase activity, acting on the CH-NH group of donors, NAD or NADP as acceptor [GO:0016646] Sources: EC:1.5.1.1, MetaCyc:PYRROLINE-2-CARBOXYLATE-REDUCTASE-RXN